{
  "term_id": "GO:0005886",
  "term_label": "plasma membrane",
  "gene_name": "Vasoactive intestinal polypeptide receptor 2",
  "gene_symbol": "VIPR2",
  "gene": "UniProtKB:P41587"
}